{
  "term_label": "retinol metabolic process",
  "gene_symbol": "RETSAT",
  "gene_name": "All-trans-retinol 13,14-reductase",
  "term_id": "GO:0042572",
  "gene": "UniProtKB:Q6NUM9"
}